{
  "gene_symbol": "PLK5",
  "gene": "UniProtKB:Q496M5",
  "term_id": "GO:2000045",
  "term_label": "regulation of G1/S transition of mitotic cell cycle",
  "gene_name": "Inactive serine_threonine-protein kinase PLK5"
}